efflux transmembrane transporter activity [GO:0015562] (molecular function) Definition: Enables the transfer of a specific substance or related group of substances from the inside of the cell to the outside of the cell across a membrane. Sources: GOC:ai, GOC:mtg_transport, ISBN:0815340729 Also known as: efflux permease activity, efflux transporter activity, monocarboxylate (lactate, pyruvate, mevalonate) uptake/efflux porter activity Subtypes: GO:0010542, nitrite efflux transmembrane transporter activity [GO:0015514], formate efflux transmembrane transporter activity [GO:0015660], silicon efflux transmembrane transporter activity [GO:0032523], GO:0034639, monoatomic cation efflux transmembrane transporter activity [GO:0046583], borate efflux transmembrane transporter activity [GO:0080139] Relationships: is a type of transmembrane transporter activity [GO:0022857]